{
  "term_id": "GO:0042998",
  "gene_name": "Consortin",
  "gene": "UniProtKB:Q6PJW8",
  "gene_symbol": "CNST",
  "term_label": "positive regulation of Golgi to plasma membrane protein transport"
}